dendritic cell apoptotic process [GO:0097048] (biological process) References: PMID:15059845 Sources: CL:0000451, GOC:BHF, GOC:mtg_apoptosis Definition: Any apoptotic process in a dendritic cell, a cell of hematopoietic origin, typically resident in particular tissues, specialized in the uptake, processing, and transport of antigens to lymph nodes for the purpose of stimulating an immune response via T cell activation. Regulation: regulated by regulation of dendritic cell apoptotic process [GO:2000668]; negatively regulated by GO:2000669; positively regulated by positive regulation of dendritic cell apoptotic process [GO:2000670] Relationships: is a type of leukocyte apoptotic process [GO:0071887] Also known as: dendritic cell apoptosis